{
  "gene_symbol": "CLIP4",
  "gene": "UniProtKB:Q8N3C7",
  "gene_name": "CAP-Gly domain-containing linker protein 4",
  "term_label": "microtubule plus-end binding",
  "term_id": "GO:0051010"
}